{
  "gene": "UniProtKB:P22309",
  "gene_symbol": "UGT1A1",
  "term_id": "GO:0004857",
  "term_label": "enzyme inhibitor activity",
  "gene_name": "UDP-glucuronosyltransferase 1A1"
}